{
  "gene": "UniProtKB:Q9Y6K5",
  "term_label": "cytosol",
  "term_id": "GO:0005829",
  "gene_name": "2'-5'-oligoadenylate synthase 3",
  "gene_symbol": "OAS3"
}